proteolysis within endosome associated with antigen processing and presentation [GO:0002499] (biological process) Definition: The hydrolysis of a peptide bond or bonds within a protein by endosomal resident proteases contributing to antigen processing and presentation. References: PMID:15771591 Sources: GOC:add, ISBN:0781735149 Also known as: endosomal proteolysis associated with antigen processing and presentation Relationships: is a type of proteolysis associated with antigen processing and presentation [GO:0002496]; occurs in endosome [GO:0005768]